{
  "gene": "UniProtKB:Q8N4C8",
  "term_label": "protein serine/threonine kinase activity",
  "gene_name": "Misshapen-like kinase 1",
  "term_id": "GO:0004674",
  "gene_symbol": "MINK1"
}